{
  "gene_name": "RUN and FYVE domain-containing protein 4",
  "gene_symbol": "RUFY4",
  "gene": "UniProtKB:Q6ZNE9",
  "term_id": "GO:0000045",
  "term_label": "autophagosome assembly"
}